{
  "gene_name": "Muscleblind-like protein 3",
  "gene": "UniProtKB:Q9NUK0",
  "term_id": "GO:0005654",
  "term_label": "nucleoplasm",
  "gene_symbol": "MBNL3"
}